{
  "term_id": "GO:0030424",
  "gene_symbol": "TMEM108",
  "term_label": "axon",
  "gene_name": "Transmembrane protein 108",
  "gene": "UniProtKB:Q6UXF1"
}